reduced coenzyme F420:heterodisulfide oxidoreductase activity [GO:0052752] (molecular function) Relationships: is a type of oxidoreductase activity, acting on a sulfur group of donors [GO:0016667] Definition: Catalysis of the reaction: reduced coenzyme F420 + CoB-S-S-CoM = coenzyme F420 + CoM-SH + CoB-SH. References: PMID:9914308 Sources: GOC:mengo_curators Also known as: F420-dependent heterodisulfide oxidoreductase activity, F420H2:heterodisulfide oxidoreductase activity, coenzyme F420-dependent heterodisulfide oxidoreductase activity